{
  "gene_name": "Histone H2B type 2-F",
  "gene": "UniProtKB:Q5QNW6",
  "gene_symbol": "H2BC18",
  "term_label": "chromatin organization",
  "term_id": "GO:0006325"
}